{
  "gene_name": "Histone-lysine N-methyltransferase SETMAR",
  "gene": "UniProtKB:Q53H47",
  "gene_symbol": "SETMAR",
  "term_id": "GO:0046975",
  "term_label": "histone H3K36 methyltransferase activity"
}